{
  "gene_name": "KRAB domain-containing protein 1",
  "gene_symbol": "KRBOX1",
  "term_label": "negative regulation of transcription by RNA polymerase II",
  "gene": "UniProtKB:C9JBD0",
  "term_id": "GO:0000122"
}